{
  "term_label": "Unknown molecular function",
  "gene_symbol": "HAPLN1",
  "gene": "UniProtKB:P10915",
  "gene_name": "Hyaluronan and proteoglycan link protein 1",
  "term_id": "UNKNOWN:0001"
}